{
  "term_label": "regulatory ncRNA-mediated post-transcriptional gene silencing",
  "gene_name": "Helicase with zinc finger domain 2",
  "gene": "UniProtKB:Q9BYK8",
  "gene_symbol": "HELZ2",
  "term_id": "GO:0035194"
}